positive regulation of N',N'',N'''-triacetylfusarinine C biosynthetic process [GO:1900697] (biological process) Definition: Any process that activates or increases the frequency, rate or extent of N',N'',N'''-triacetylfusarinine C biosynthetic process. Also known as: activation of N',N'',N'''-triacetylfusarinine C anabolism, activation of N',N'',N'''-triacetylfusarinine C biosynthesis, activation of N',N'',N'''-triacetylfusarinine C formation, activation of N',N'',N'''-triacetylfusarinine C synthesis, positive regulation of N',N'',N'''-triacetylfusarinine C anabolism, positive regulation of N',N'',N'''-triacetylfusarinine C biosynthesis, positive regulation of N',N'',N'''-triacetylfusarinine C formation, positive regulation of N',N'',N'''-triacetylfusarinine C synthesis, up regulation of N',N'',N'''-triacetylfusarinine C anabolism, up regulation of N',N'',N'''-triacetylfusarinine C biosynthesis, up regulation of N',N'',N'''-triacetylfusarinine C biosynthetic process, up regulation of N',N'',N'''-triacetylfusarinine C formation, up regulation of N',N'',N'''-triacetylfusarinine C synthesis, up-regulation of N',N'',N'''-triacetylfusarinine C anabolism, up-regulation of N',N'',N'''-triacetylfusarinine C biosynthesis, up-regulation of N',N'',N'''-triacetylfusarinine C biosynthetic process, up-regulation of N',N'',N'''-triacetylfusarinine C formation, up-regulation of N',N'',N'''-triacetylfusarinine C synthesis, upregulation of N',N'',N'''-triacetylfusarinine C anabolism, upregulation of N',N'',N'''-triacetylfusarinine C biosynthesis, upregulation of N',N'',N'''-triacetylfusarinine C biosynthetic process, upregulation of N',N'',N'''-triacetylfusarinine C formation, upregulation of N',N'',N'''-triacetylfusarinine C synthesis, activation of N',N'',N'''-triacetylfusarinine C biosynthetic process Relationships: is a type of positive regulation of secondary metabolite biosynthetic process [GO:1900378]; is a type of regulation of N',N'',N'''-triacetylfusarinine C biosynthetic process [GO:1900695]; positively regulates GO:1900551 Sources: GOC:TermGenie, GOC:di